{
  "term_id": "UNKNOWN:0003",
  "gene_name": "G patch domain-containing protein 3",
  "gene_symbol": "GPATCH3",
  "gene": "UniProtKB:Q96I76",
  "term_label": "Unknown cellular component"
}